{
  "gene": "UniProtKB:Q13107",
  "term_label": "Unknown biological process",
  "gene_symbol": "USP4",
  "term_id": "UNKNOWN:0002",
  "gene_name": "Ubiquitin carboxyl-terminal hydrolase 4"
}